venom-mediated depletion of circulating fibrinogen [GO:0044536] (biological process) Relationships: is a type of GO:0044483 Also known as: envenomation resulting in depletion of circulating fibrinogen, envenomation resulting in depletion of circulating fibrinogen in another organism, envenomation resulting in depletion of circulating fibrinogen in other organism, envenomation resulting in negative regulation of circulating fibrinogen in other organism Definition: The process which begins with venom being forced into an organism by the bite or sting of another organism, and ends with a reduction in the quantity of fibrinogen found in the bloodstream of the bitten/stung organism. References: PMID:21130897 Sources: GOC:fj, GOC:jl Subtypes: venom-mediated fibrinogenolysis [GO:0044485]